{
  "gene_name": "Inactive peptidyl-prolyl cis-trans isomerase FKBP6",
  "term_label": "cytoplasm",
  "term_id": "GO:0005737",
  "gene_symbol": "FKBP6",
  "gene": "UniProtKB:O75344"
}